{
  "gene": "UniProtKB:O43781",
  "gene_symbol": "DYRK3",
  "term_id": "GO:0035617",
  "term_label": "stress granule disassembly",
  "gene_name": "Dual specificity tyrosine-phosphorylation-regulated kinase 3"
}